positive regulation of phytoalexin biosynthetic process [GO:0052322] (biological process) Relationships: is a type of defense response to symbiont [GO:0140546]; is a type of positive regulation of secondary metabolite biosynthetic process [GO:1900378]; positively regulates phytoalexin biosynthetic process [GO:0052315] Definition: Any process that activates, maintains or increases the frequency, rate or extent of phytoalexin biosynthesis, the chemical reactions and pathways resulting in the formation of phytoalexins. Sources: GOC:mtg_pamgo_17jul06 Also known as: positive regulation of phytoalexin biosynthesis, up regulation of phytoalexin biosynthesis, up-regulation of phytoalexin biosynthesis, upregulation of phytoalexin biosynthesis, activation of phytoalexin biosynthesis, stimulation of phytoalexin biosynthesis Subtypes: GO:1901183